CD40 receptor binding [GO:0005174] (molecular function) Definition: Binding to CD40, a receptor found on the surface of all B-lymphocytes. Relationships: is a type of tumor necrosis factor receptor superfamily binding [GO:0032813] Sources: GOC:jl, ISBN:0120781859